{
  "gene_symbol": "HADHB",
  "term_label": "fatty acid beta-oxidation",
  "gene_name": "Trifunctional enzyme subunit beta, mitochondrial",
  "term_id": "GO:0006635",
  "gene": "UniProtKB:P55084"
}